olfactory receptor binding [GO:0031849] (molecular function) Sources: GOC:mah, GOC:nln Definition: Binding to an olfactory receptor. Relationships: is a type of G protein-coupled receptor binding [GO:0001664] Also known as: olfactory receptor ligand